{
  "gene": "UniProtKB:O43915",
  "term_label": "growth factor activity",
  "term_id": "GO:0008083",
  "gene_symbol": "VEGFD",
  "gene_name": "Vascular endothelial growth factor D"
}